{
  "term_label": "ubiquitin protein ligase activity",
  "term_id": "GO:0061630",
  "gene_name": "Tripartite motif-containing protein 43",
  "gene": "UniProtKB:Q96BQ3",
  "gene_symbol": "TRIM43"
}